{
  "term_id": "GO:0003697",
  "gene_name": "Replication protein A 32 kDa subunit",
  "term_label": "single-stranded DNA binding",
  "gene": "UniProtKB:P15927",
  "gene_symbol": "RPA2"
}